{
  "term_label": "alpha-(1->3)-fucosyltransferase activity",
  "gene_name": "Alpha-(1,3)-fucosyltransferase 10",
  "gene": "UniProtKB:Q6P4F1",
  "gene_symbol": "FUT10",
  "term_id": "GO:0046920"
}